{
  "gene_name": "Keratin, type I cuticular Ha8",
  "term_label": "keratin filament",
  "gene_symbol": "KRT38",
  "term_id": "GO:0045095",
  "gene": "UniProtKB:O76015"
}